{
  "term_label": "BRCA1-A complex",
  "gene_symbol": "BRCA1",
  "gene": "UniProtKB:P38398",
  "gene_name": "Breast cancer type 1 susceptibility protein",
  "term_id": "GO:0070531"
}